{
  "gene": "UniProtKB:P48023",
  "term_id": "GO:2001238",
  "gene_symbol": "FASLG",
  "term_label": "positive regulation of extrinsic apoptotic signaling pathway",
  "gene_name": "Tumor necrosis factor ligand superfamily member 6"
}